{
  "gene_name": "Rho-related GTP-binding protein RhoQ",
  "term_label": "actin filament organization",
  "gene_symbol": "RHOQ",
  "gene": "UniProtKB:P17081",
  "term_id": "GO:0007015"
}